progesterone catabolic process [GO:0006709] (biological process) Relationships: is a type of C21-steroid hormone catabolic process [GO:0008208]; is a type of GO:0042182; is a type of progesterone metabolic process [GO:0042448]; is a type of olefinic compound catabolic process [GO:0120256] References: PMID:11392024 Sources: GOC:jl Also known as: progesterone breakdown, progesterone catabolism, progesterone degradation Definition: The chemical reactions and pathways resulting in the breakdown of progesterone, a steroid hormone produced in the ovary which prepares and maintains the uterus for pregnancy. Also found in plants.